sperm plasma membrane disassembly [GO:0035045] (biological process) Sources: GOC:bf, ISBN:0879694238 Relationships: is a type of plasma membrane organization [GO:0007009]; is a type of cellular process involved in reproduction in multicellular organism [GO:0022412]; is a type of membrane disassembly [GO:0030397]; BFO_0000050 single fertilization [GO:0007338] Also known as: sperm plasma membrane breakdown, sperm plasma membrane catabolism, sperm plasma membrane degradation Definition: The gradual disintegration of the sperm plasma membrane following insemination. This process is seen in Drosophila after entry of the entire sperm, surrounded by its plasma membrane, into the egg.